{
  "gene_symbol": "PTX3",
  "gene_name": "Pentraxin-related protein PTX3",
  "gene": "UniProtKB:P26022",
  "term_id": "GO:0044793",
  "term_label": "host-mediated suppression of viral proces"
}